{
  "gene_name": "Neutral ceramidase",
  "gene": "UniProtKB:Q9NR71",
  "term_label": "N-acylsphingosine amidohydrolase activity",
  "term_id": "GO:0017040",
  "gene_symbol": "ASAH2"
}